{
  "term_label": "regulation of myeloid cell differentiation",
  "gene_name": "Transcription factor MafB",
  "gene_symbol": "MAFB",
  "term_id": "GO:0045637",
  "gene": "UniProtKB:Q9Y5Q3"
}